{
  "gene_symbol": "NAT10",
  "gene": "UniProtKB:Q9H0A0",
  "term_label": "18S rRNA cytidine N-acetyltransferase activity",
  "term_id": "GO:1990883",
  "gene_name": "RNA cytidine acetyltransferase"
}